{
  "term_label": "receptor complex",
  "gene_symbol": "MST1R",
  "gene": "UniProtKB:Q04912",
  "term_id": "GO:0043235",
  "gene_name": "Macrophage-stimulating protein receptor"
}